{
  "gene_symbol": "OPTN",
  "gene_name": "Optineurin",
  "term_label": "nucleus",
  "gene": "UniProtKB:Q96CV9",
  "term_id": "GO:0005634"
}